{
  "gene_symbol": "EDA2R",
  "gene": "UniProtKB:Q9HAV5",
  "gene_name": "Tumor necrosis factor receptor superfamily member 27",
  "term_label": "signaling receptor activity",
  "term_id": "GO:0038023"
}